{
  "term_id": "GO:0008184",
  "gene_symbol": "PYGL",
  "gene": "UniProtKB:P06737",
  "term_label": "glycogen phosphorylase activity",
  "gene_name": "Glycogen phosphorylase, liver form"
}